{
  "gene": "UniProtKB:Q8N8F6",
  "gene_symbol": "YIPF7",
  "term_id": "UNKNOWN:0001",
  "gene_name": "Protein YIPF7",
  "term_label": "Unknown molecular function"
}